{
  "gene_symbol": "GCM2",
  "gene_name": "Chorion-specific transcription factor GCMb",
  "gene": "UniProtKB:O75603",
  "term_label": "DNA-binding transcription factor activity, RNA polymerase II-specific",
  "term_id": "GO:0000981"
}